{
  "gene_symbol": "TRMT2B",
  "term_id": "UNKNOWN:0003",
  "gene_name": "tRNA (uracil-5-)-methyltransferase homolog B",
  "term_label": "Unknown cellular component",
  "gene": "UniProtKB:Q96GJ1"
}